{
  "gene_name": "Protein NDRG1",
  "term_id": "UNKNOWN:0001",
  "term_label": "Unknown molecular function",
  "gene": "UniProtKB:Q92597",
  "gene_symbol": "NDRG1"
}